{
  "gene_symbol": "KDELR3",
  "term_label": "cis-Golgi network",
  "term_id": "GO:0005801",
  "gene": "UniProtKB:O43731",
  "gene_name": "ER lumen protein-retaining receptor 3"
}